{
  "term_id": "GO:0001963",
  "term_label": "synaptic transmission, dopaminergic",
  "gene_symbol": "TH",
  "gene": "UniProtKB:P07101",
  "gene_name": "Tyrosine 3-monooxygenase"
}